basal ectoplasmic specialization [GO:0061832] (cellular component) Also known as: basal ES Relationships: is a type of GO:0005911 References: PMID:22332112, PMID:23546604 Sources: GOC:aruk, GOC:bc, GOC:dph Definition: Testis-specific junction between mature Sertoli cells involved in establishing the blood-testis barrier of the Sertoli cell.